{
  "term_id": "GO:0048471",
  "term_label": "perinuclear region of cytoplasm",
  "gene": "UniProtKB:Q6ZRF8",
  "gene_symbol": "RNF207",
  "gene_name": "RING finger protein 207"
}